{
  "term_label": "Unknown molecular function",
  "term_id": "UNKNOWN:0001",
  "gene_symbol": "CLLU1-AS1",
  "gene": "UniProtKB:Q5K130",
  "gene_name": "Putative uncharacterized protein CLLU1-AS1"
}